{
  "gene": "UniProtKB:Q9NPZ5",
  "gene_symbol": "B3GAT2",
  "gene_name": "Galactosylgalactosylxylosylprotein 3-beta-glucuronosyltransferase 2",
  "term_label": "chondroitin sulfate proteoglycan biosynthetic process",
  "term_id": "GO:0050650"
}